L-asparagine biosynthetic process from cysteine [GO:0019267] (biological process) Also known as: asparagine anabolism from cysteine, asparagine formation from cysteine, asparagine synthesis from cysteine Relationships: is a type of cysteine metabolic process [GO:0006534]; is_a L-asparagine biosynthetic process [GO:0070981] Sources: GOC:go_curators Definition: The chemical reactions and pathways resulting in the formation of asparagine from other compounds, including cysteine.